{
  "gene_symbol": "SLC35E2B",
  "gene_name": "Solute carrier family 35 member E2B",
  "term_label": "Golgi apparatus",
  "term_id": "GO:0005794",
  "gene": "UniProtKB:P0CK96"
}